{
  "gene": "UniProtKB:Q7Z6L1",
  "term_label": "lysosomal membrane",
  "gene_name": "Tectonin beta-propeller repeat-containing protein 1",
  "gene_symbol": "TECPR1",
  "term_id": "GO:0005765"
}